{
  "gene_symbol": "FOXB2",
  "gene": "UniProtKB:Q5VYV0",
  "term_id": "GO:0006357",
  "gene_name": "Forkhead box protein B2",
  "term_label": "regulation of transcription by RNA polymerase II"
}